{
  "gene": "UniProtKB:E2RYF7",
  "gene_name": "Protein PBMUCL2",
  "term_label": "Unknown biological process",
  "term_id": "UNKNOWN:0002",
  "gene_symbol": "HCG22"
}